L-lysine transmembrane transport [GO:1903401] (biological process) References: PMID:8195186 Sources: GOC:TermGenie, GOC:krc, GO_REF:0000069 Definition: The directed movement of L-lysine across a membrane. Subtypes: L-lysine transmembrane export from vacuole [GO:0089707], L-lysine transmembrane import into vacuole [GO:0090517], L-lysine import across plasma membrane [GO:0097639], GO:0160256 Relationships: is a type of L-lysine transport [GO:1902022]; is a type of L-alpha-amino acid transmembrane transport [GO:1902475]